{
  "term_id": "GO:0009986",
  "gene": "UniProtKB:O60895",
  "gene_name": "Receptor activity-modifying protein 2",
  "gene_symbol": "RAMP2",
  "term_label": "cell surface"
}